positive regulation of Kit signaling pathway [GO:1900236] (biological process) Definition: Any process that activates or increases the frequency, rate or extent of Kit signaling pathway. Also known as: activation of stem cell factor receptor signaling pathway, activation of stem cell factor signaling pathway, positive regulation of Kit signalling pathway, positive regulation of stem cell factor receptor signaling pathway, positive regulation of stem cell factor signaling pathway, up regulation of Kit signaling pathway, up regulation of stem cell factor receptor signaling pathway, up regulation of stem cell factor signaling pathway, up-regulation of Kit signaling pathway, up-regulation of stem cell factor receptor signaling pathway, up-regulation of stem cell factor signaling pathway, upregulation of Kit signaling pathway, upregulation of stem cell factor receptor signaling pathway, upregulation of stem cell factor signaling pathway, activation of Kit signaling pathway Sources: GOC:TermGenie, GOC:signaling Relationships: is a type of positive regulation of cytokine-mediated signaling pathway [GO:0001961]; is a type of regulation of Kit signaling pathway [GO:1900234]; positively regulates Kit signaling pathway [GO:0038109]